{
  "gene_name": "GAS2-like protein 3",
  "term_label": "Unknown cellular component",
  "gene": "UniProtKB:Q86XJ1",
  "gene_symbol": "GAS2L3",
  "term_id": "UNKNOWN:0003"
}